nucleotide metabolic process [GO:0009117] (biological process) Also known as: nucleotide metabolism Sources: GOC:ma Relationships: is a type of GO:0006753 Definition: The chemical reactions and pathways involving a nucleotide, a nucleoside that is esterified with (ortho)phosphate or an oligophosphate at any hydroxyl group on the glycose moiety; may be mono-, di- or triphosphate; this definition includes cyclic nucleotides (nucleoside cyclic phosphates). Regulation: regulated by regulation of nucleotide metabolic process [GO:0006140]; negatively regulated by GO:0045980; positively regulated by positive regulation of nucleotide metabolic process [GO:0045981] Subtypes: GO:0006163, GO:0006220, nucleotide biosynthetic process [GO:0009165], nucleotide catabolic process [GO:0009166], cyclic nucleotide metabolic process [GO:0009187], ribonucleotide metabolic process [GO:0009259], GO:0009262, GO:0015959, GO:0046496, flavin adenine dinucleotide metabolic process [GO:0072387], GO:0106044